regulation of protein deacetylation [GO:0090311] (biological process) Definition: Any process that modulates the rate, frequency, or extent of protein deacetylation, the removal of an acetyl group from a protein amino acid. An acetyl group is CH3CO-, derived from acetic [ethanoic] acid. Subtypes: regulation of tubulin deacetylation [GO:0090043], positive regulation of protein deacetylation [GO:0090312] Also known as: regulation of protein amino acid deacetylation Relationships: is a type of regulation of protein modification process [GO:0031399]; regulates protein deacetylation [GO:0006476] Sources: GOC:tb